endoplasmic reticulum signal peptide binding [GO:0030942] (molecular function) Relationships: is_a signal sequence binding [GO:0005048] Sources: GOC:mah Definition: Binding to an endoplasmic reticulum signal peptide, a specific peptide sequence that acts as a signal to localize the protein within the endoplasmic reticulum. Also known as: ER signal peptide binding